oocyte dorsal/ventral axis specification [GO:0007310] (BP) Sources: GOC:mtg_sensu, ISBN:0879694238 Definition: The establishment, maintenance and elaboration of the dorsal/ventral axis of the oocyte. An example of this is found in Drosophila melanogaster. Also known as: oocyte dorsal-ventral axis specification, oocyte dorsoventral axis specification, oocyte dorsal/ventral axis determination Relationships: is a type of oocyte axis specification [GO:0007309]; is a type of dorsal/ventral axis specification [GO:0009950] Subtypes: maternal specification of dorsal/ventral axis, oocyte, germ-line encoded [GO:0007311], GO:0007313